{
  "term_id": "UNKNOWN:0003",
  "term_label": "Unknown cellular component",
  "gene_name": "Transmembrane protein 220",
  "gene": "UniProtKB:Q6QAJ8",
  "gene_symbol": "TMEM220"
}